{
  "gene": "UniProtKB:O94804",
  "term_id": "GO:0005737",
  "gene_symbol": "STK10",
  "gene_name": "Serine_threonine-protein kinase 10",
  "term_label": "cytoplasm"
}